{
  "gene": "UniProtKB:O15231",
  "gene_name": "Zinc finger protein 185",
  "term_label": "Unknown cellular component",
  "term_id": "UNKNOWN:0003",
  "gene_symbol": "ZNF185"
}